biofilm matrix disassembly [GO:0098786] (biological process) Definition: A process that results in the disassembly of a biofilm matrix. Sources: GOC:mah Relationships: is a type of extracellular matrix disassembly [GO:0022617]; is a type of biofilm matrix organization [GO:0098784]